lumenal side of medial-Golgi cisterna membrane [GO:0160280] (cellular component) Definition: The membrane leaflet of the medial-Golgi cisternae that directly contacts the Golgi lumen, hosts glycosyltransferases and enzymes to modify N-linked oligosaccharides by trimming mannose and adding N-acetylglucosamine. Also known as: lumenal face of medial-Golgi cisterna membrane, lumenal leaflet of Golgi medial cisterna membrane Relationships: is a type of lumenal side of membrane [GO:0098576]; is part of Golgi medial cisterna membrane [GO:1990675] References: PMID:28777890, PMID:34597626, PMID:36658747, PMID:39331042